oxidoreductase activity, acting on CH or CH2 groups [GO:0016725] (molecular function) Subtypes: oxidoreductase activity, acting on CH or CH2 groups, NAD or NADP as acceptor [GO:0016726], oxidoreductase activity, acting on CH or CH2 groups, oxygen as acceptor [GO:0016727], oxidoreductase activity, acting on CH or CH2 groups, disulfide as acceptor [GO:0016728], ethylbenzene hydroxylase activity [GO:0018693], 4-cresol dehydrogenase (hydroxylating) activity [GO:0018695], oxidoreductase activity, acting on CH or CH2 groups, quinone or similar compound as acceptor [GO:0033695], GO:0033791, formate dehydrogenase (coenzyme F420) activity [GO:0043794], uracil dehydrogenase activity [GO:0050383], oxidoreductase activity, acting on CH or CH2 groups, with an iron-sulfur protein as acceptor [GO:0052592], GO:0052620, epoxyqueuosine reductase activity [GO:0052693], GO:0120547 Sources: GOC:ai Definition: Catalysis of an oxidation-reduction (redox) reaction in which a CH2 group acts as a hydrogen or electron donor and reduces a hydrogen or electron acceptor. Also known as: oxidoreductase activity, acting on CH or CH2 groups, other acceptors Relationships: is a type of oxidoreductase activity [GO:0016491]